{
  "gene_symbol": "IL25",
  "term_id": "UNKNOWN:0001",
  "gene_name": "Interleukin-25",
  "gene": "UniProtKB:Q9H293",
  "term_label": "Unknown molecular function"
}